{
  "gene_name": "T cell receptor alpha joining 29 (Fragment)",
  "term_label": "Unknown cellular component",
  "term_id": "UNKNOWN:0003",
  "gene": "UniProtKB:A0A075B711",
  "gene_symbol": "TRAJ29"
}